{
  "term_id": "GO:0004719",
  "term_label": "protein-L-isoaspartate (D-aspartate) O-methyltransferase activity",
  "gene_name": "Protein-L-isoaspartate(D-aspartate) O-methyltransferase",
  "gene_symbol": "PCMT1",
  "gene": "UniProtKB:P22061"
}